NuA3 histone acetyltransferase complex [GO:0033100] (CC) Subtypes: NuA3a histone acetyltransferase complex [GO:1990467], NuA3b histone acetyltransferase complex [GO:1990468] Definition: A Gcn5-independent multisubunit complex that catalyzes the acetylation of histone H3. The budding yeast complex includes Sas3p, Taf30p, and Yng1p. Relationships: is a type of GO:0070775 References: PMID:10817755, PMID:17157260